{
  "term_id": "GO:0030280",
  "gene": "UniProtKB:P12035",
  "gene_symbol": "KRT3",
  "term_label": "structural constituent of skin epidermis",
  "gene_name": "Keratin, type II cytoskeletal 3"
}